type 6 serotonin receptor binding [GO:0031832] (molecular function) Also known as: 5-hydroxytryptamine 6 receptor binding, type 6 serotonin receptor ligand Sources: GOC:mah, GOC:nln Relationships: is a type of G protein-coupled serotonin receptor binding [GO:0031821] Definition: Binding to a type 6 serotonin receptor.